{
  "gene_name": "T cell receptor alpha joining 32 (Fragment)",
  "gene": "UniProtKB:A0A075B6X3",
  "term_id": "UNKNOWN:0003",
  "term_label": "Unknown cellular component",
  "gene_symbol": "TRAJ32"
}